{
  "term_id": "GO:0000056",
  "term_label": "ribosomal small subunit export from nucleus",
  "gene": "UniProtKB:Q86U38",
  "gene_name": "Nucleolar protein 9",
  "gene_symbol": "NOP9"
}